{
  "term_id": "GO:0005634",
  "term_label": "nucleus",
  "gene_symbol": "ADPRS",
  "gene": "UniProtKB:Q9NX46",
  "gene_name": "ADP-ribosylhydrolase ARH3"
}